{
  "gene_name": "Protein flightless-1 homolog",
  "term_id": "GO:0005634",
  "gene": "UniProtKB:Q13045",
  "term_label": "nucleus",
  "gene_symbol": "FLII"
}